{
  "gene_symbol": "HES5",
  "gene": "UniProtKB:Q5TA89",
  "term_label": "negative regulation of transcription by RNA polymerase II",
  "gene_name": "Transcription factor HES-5",
  "term_id": "GO:0000122"
}